{
  "term_id": "UNKNOWN:0003",
  "gene_name": "Putative uncharacterized protein C2orf48",
  "term_label": "Unknown cellular component",
  "gene": "UniProtKB:Q96LS8",
  "gene_symbol": "C2orf48"
}